{
  "gene_symbol": "DLX2",
  "gene": "UniProtKB:Q07687",
  "term_label": "DNA-binding transcription factor activity, RNA polymerase II-specific",
  "gene_name": "Homeobox protein DLX-2",
  "term_id": "GO:0000981"
}